blood coagulation, intrinsic pathway [GO:0007597] (biological process) Regulation: regulated by regulation of blood coagulation, intrinsic pathway [GO:2000266]; negatively regulated by negative regulation of blood coagulation, intrinsic pathway [GO:2000267]; positively regulated by positive regulation of blood coagulation, intrinsic pathway [GO:2000268] Definition: A protein activation cascade that initiates blood coagulation, triggered when Factor XII, prekallikrein (PK) and high-molecular-weight kininogen  (HK) assemble on a suitable surface or polymer. This results in the reciprocal activation of factor XII to Factor XIIa by kallikrein, and PK to kallikrein by Factor XIIa. The resulting generation of Factor XIIa activates Factor XI to Factor XIa, which then converts Factor IX to Factor IXa. Factor IXa converts Factor X to Xa. Factor Xa then initiates the common pathway. Note: See also the biological process term 'blood coagulation, extrinsic pathway ; GO:0007598' and 'blood coagulation, common pathway ; GO:0072377'. Also known as: initiation of blood coagulation cascade, contact activation system, initiation of blood coagulation cascade, contact pathway References: PMID:26018600 Sources: GOC:add, GOC:mah, GOC:pde Relationships: is a type of GO:0072376; is part of GO:0072378